{
  "gene_symbol": "SHROOM2",
  "term_label": "apical junction complex",
  "gene_name": "Protein Shroom2",
  "term_id": "GO:0043296",
  "gene": "UniProtKB:Q13796"
}